{
  "term_label": "plasma membrane",
  "gene_name": "Killer cell lectin-like receptor subfamily B member 1",
  "gene_symbol": "KLRB1",
  "gene": "UniProtKB:Q12918",
  "term_id": "GO:0005886"
}